anterograde trans-synaptic signaling by trans-synaptic protein complex [GO:0098941] (biological process) Sources: GOC:dos Definition: Cell-cell signaling from presynapse to postynapse, across the synaptic cleft, mediated by a trans-synaptic protein complex. Relationships: is a type of anterograde trans-synaptic signaling [GO:0098916]; is a type of GO:0099545